negative regulation of ribosomal protein gene transcription by RNA polymerase II [GO:0010688] (biological process) Relationships: is a type of GO:0000122; is a type of GO:0060962 Sources: GOC:dph, GOC:tb, GOC:txnOH Subtypes: GO:0010689, GO:0010690, negative regulation of ribosomal protein gene transcription from RNA polymerase II promoter in response to nutrient levels [GO:0010691] Also known as: negative regulation of ribosomal protein gene transcription from RNA polymerase II promoter Definition: Any process that decreases the frequency, rate or extent of the synthesis of RNA from ribosomal protein genes mediated by RNA polymerase II.